{
  "gene_name": "Cilia- and flagella-associated protein 410",
  "gene_symbol": "CFAP410",
  "term_id": "UNKNOWN:0003",
  "gene": "UniProtKB:O43822",
  "term_label": "Unknown cellular component"
}